TRC complex [GO:0072380] (cellular component) References: PMID:20850366, PMID:23142665 Sources: GOC:mah Also known as: TMD recognition complex, GET4-GET5 transmembrane domain recognition complex Definition: A protein complex found in yeast that contains GET4, MDY2 (GET5), SGT2, and at least two heat shock proteins, HSP104 and YBR137W. The TRC complex transfers tail-anchored (TA) proteins to GET3 for targeting to the endoplasmic reticulum membrane. Relationships: is a type of ER membrane insertion complex [GO:0072379]